{
  "term_id": "GO:0045048",
  "gene": "UniProtKB:Q15629",
  "gene_symbol": "TRAM1",
  "term_label": "protein insertion into ER membrane",
  "gene_name": "Translocating chain-associated membrane protein 1"
}